{
  "gene_symbol": "GMPPB",
  "term_id": "GO:0004475",
  "term_label": "mannose-1-phosphate guanylyltransferase (GTP) activity",
  "gene_name": "Mannose-1-phosphate guanyltransferase beta",
  "gene": "UniProtKB:Q9Y5P6"
}